{
  "term_label": "plasma membrane",
  "gene_name": "Leucine-rich repeat and immunoglobulin-like domain-containing nogo receptor-interacting protein 1",
  "gene_symbol": "LINGO1",
  "gene": "UniProtKB:Q96FE5",
  "term_id": "GO:0005886"
}